negative regulation of leucophore differentiation [GO:0048776] (biological process) Definition: Any process that stops, prevents, or reduces the frequency, rate or extent of leucophore differentiation. Also known as: down regulation of leucophore differentiation, down-regulation of leucophore differentiation, downregulation of leucophore differentiation, inhibition of leucophore differentiation Relationships: is a type of GO:0048775; is a type of GO:0050941; negatively regulates leucophore differentiation [GO:0048772] Sources: GOC:mh